{
  "gene": "UniProtKB:Q15392",
  "term_label": "cytoplasm",
  "gene_symbol": "DHCR24",
  "term_id": "GO:0005737",
  "gene_name": "Delta(24)-sterol reductase"
}